negative regulation of collagen biosynthetic process [GO:0032966] (biological process) Definition: Any process that stops, prevents, or reduces the frequency, rate or extent of the chemical reactions and pathways resulting in the formation of collagen, any of a group of fibrous proteins of very high tensile strength that form the main component of connective tissue in animals. Sources: GOC:mah Relationships: is a type of negative regulation of biosynthetic process [GO:0009890]; is_a negative regulation of collagen metabolic process [GO:0010713]; is a type of regulation of collagen biosynthetic process [GO:0032965]; negatively regulates GO:0032964 Also known as: negative regulation of collagen anabolism, negative regulation of collagen biosynthesis, negative regulation of collagen formation, negative regulation of collagen synthesis